{
  "term_id": "UNKNOWN:0003",
  "gene_name": "Ankyrin repeat domain-containing protein 50",
  "gene_symbol": "ANKRD50",
  "gene": "UniProtKB:Q9ULJ7",
  "term_label": "Unknown cellular component"
}